{
  "gene_symbol": "WASHC1",
  "gene_name": "WASH complex subunit 1",
  "term_id": "GO:0055037",
  "term_label": "recycling endosome",
  "gene": "UniProtKB:A8K0Z3"
}